{
  "gene": "UniProtKB:Q8NHY5",
  "term_label": "site of double-strand break",
  "gene_symbol": "HUS1B",
  "gene_name": "Checkpoint protein HUS1B",
  "term_id": "GO:0035861"
}